coronal suture morphogenesis [GO:0060365] (biological process) Definition: The process in which the coronal suture is generated and organized. Sources: GOC:dph, GOC:sl Relationships: is a type of cranial suture morphogenesis [GO:0060363]